{
  "gene_name": "Alcohol dehydrogenase 1A",
  "gene_symbol": "ADH1A",
  "term_label": "all-trans-retinol dehydrogenase (NAD+) activity",
  "term_id": "GO:0004745",
  "gene": "UniProtKB:P07327"
}